{
  "gene": "UniProtKB:Q6ZUI0",
  "term_id": "GO:0005737",
  "gene_name": "Tumor protein p63-regulated gene 1 protein",
  "term_label": "cytoplasm",
  "gene_symbol": "TPRG1"
}